DNA strand invasion [GO:0042148] (biological process) Definition: The process in which the nucleoprotein complex (composed of the broken single-strand DNA and the recombinase) searches and identifies a region of homology in intact duplex DNA. The broken single-strand DNA displaces the like strand and forms Watson-Crick base pairs with its complement, forming a duplex in which each strand is from one of the two recombining DNA molecules. References: PMID:10357855 Sources: GOC:elh Subtypes: meiotic strand invasion [GO:0000708] Relationships: is a type of DNA metabolic process [GO:0006259]; is part of DNA recombination [GO:0006310] Also known as: Rad51-mediated strand invasion, strand invasion, D-loop biosynthesis, D-loop formation, displacement loop biosynthesis, displacement loop formation Regulation: regulated by GO:0060542; negatively regulated by negative regulation of strand invasion [GO:0060543]; positively regulated by positive regulation of strand invasion [GO:0098530]